{
  "term_label": "paranode region of axon",
  "gene_symbol": "NCMAP",
  "gene": "UniProtKB:Q5T1S8",
  "term_id": "GO:0033270",
  "gene_name": "Noncompact myelin-associated protein"
}